{
  "term_label": "guanyl-nucleotide exchange factor activity",
  "gene": "UniProtKB:A1IGU5",
  "gene_name": "Rho guanine nucleotide exchange factor 37",
  "term_id": "GO:0005085",
  "gene_symbol": "ARHGEF37"
}